{
  "term_label": "intracellular receptor signaling pathway",
  "gene": "UniProtKB:P20393",
  "term_id": "GO:0030522",
  "gene_name": "Nuclear receptor subfamily 1 group D member 1",
  "gene_symbol": "NR1D1"
}